{
  "gene": "UniProtKB:A7XYQ1",
  "term_label": "inner ear morphogenesis",
  "term_id": "GO:0042472",
  "gene_symbol": "SOBP",
  "gene_name": "Sine oculis-binding protein homolog"
}